{
  "term_id": "GO:0043235",
  "gene": "UniProtKB:Q68DU8",
  "term_label": "receptor complex",
  "gene_name": "BTB_POZ domain-containing protein KCTD16",
  "gene_symbol": "KCTD16"
}